{
  "gene_name": "Arachidonate 12-lipoxygenase, 12R-type",
  "term_label": "lipoxygenase pathway",
  "gene": "UniProtKB:O75342",
  "term_id": "GO:0019372",
  "gene_symbol": "ALOX12B"
}